{
  "term_id": "GO:0017183",
  "term_label": "protein histidyl modification to diphthamide",
  "gene_symbol": "DPH3P1",
  "gene": "UniProtKB:Q9H4G8",
  "gene_name": "Putative DPH3 homolog B"
}